{
  "gene": "UniProtKB:O14514",
  "gene_name": "Adhesion G protein-coupled receptor B1",
  "gene_symbol": "ADGRB1",
  "term_label": "G protein-coupled receptor signaling pathway",
  "term_id": "GO:0007186"
}